cold acclimation [GO:0009631] (biological process) Relationships: is a type of response to cold [GO:0009409] Definition: Any process that increases freezing tolerance of an organism in response to low, nonfreezing temperatures. Sources: GOC:syr